sucrose import across plasma membrane [GO:0106082] (biological process) Definition: The directed movement of sucrose from outside of a cell, across the plasma membrane and into the cytosol. Relationships: is a type of carbohydrate import across plasma membrane [GO:0098704]; is a type of GO:1904982 References: PMID:11136464